{
  "gene_symbol": "APBB1IP",
  "gene": "UniProtKB:Q7Z5R6",
  "term_id": "GO:0005829",
  "term_label": "cytosol",
  "gene_name": "Amyloid beta A4 precursor protein-binding family B member 1-interacting protein"
}